{
  "gene_name": "Annexin A5",
  "term_label": "vesicle membrane",
  "term_id": "GO:0012506",
  "gene": "UniProtKB:P08758",
  "gene_symbol": "ANXA5"
}